{
  "term_id": "GO:0006357",
  "gene": "UniProtKB:P26367",
  "gene_name": "Paired box protein Pax-6",
  "term_label": "regulation of transcription by RNA polymerase II",
  "gene_symbol": "PAX6"
}